regulation of cell activation [GO:0050865] (biological process) Definition: Any process that modulates the frequency, rate or extent of cell activation, the change in the morphology or behavior of a cell resulting from exposure to an activating factor such as a cellular or soluble ligand. Relationships: is a type of GO:0050794; is a type of regulation of multicellular organismal process [GO:0051239]; regulates GO:0001775 Sources: GOC:ai Subtypes: GO:0002694, GO:0010543, regulation of satellite cell activation involved in skeletal muscle regeneration [GO:0014717], negative regulation of cell activation [GO:0050866], positive regulation of cell activation [GO:0050867], GO:0060472, GO:0061888, GO:1904987, regulation of hepatic stellate cell activation [GO:2000489]